histone H1 demethylase activity [GO:0160243] (molecular function) Relationships: is a type of histone demethylase activity [GO:0032452] References: PMID:19144645 Definition: Catalysis of the removal of a methyl group from a modified lysine residue of the histone H1 protein. This is a dioxygenase reaction that is dependent on Fe(II) and 2-oxoglutarate.